T=9 icosahedral viral capsid [GO:0160168] (cellular component) Relationships: is_a GO:0019030 Definition: The protein coat that surrounds the infective nucleic acid in some virus particles where the subunits (capsomeres) are arranged to form an icosahedron with T=9 symmetry. The T=9 capsid is composed of 12 pentameric and 80 hexameric capsomeres. References: PMID:37138077